regulation of synaptic membrane adhesion [GO:0099179] (biological process) Also known as: regulation of synapse adhesion between pre- and post-synapse Sources: GOC:dos Definition: Any process that modulates the frequency, rate or extent of adhesion between pre- and post-synaptic membranes. Relationships: is a type of regulation of cell-cell adhesion [GO:0022407]; is a type of GO:0050807; regulates synaptic membrane adhesion [GO:0099560]